{
  "term_id": "GO:0005634",
  "gene_name": "Testis-specific Y-encoded protein 4",
  "gene_symbol": "TSPY4",
  "gene": "UniProtKB:P0CV99",
  "term_label": "nucleus"
}